{
  "gene": "UniProtKB:P61009",
  "term_label": "protein targeting to ER",
  "term_id": "GO:0045047",
  "gene_symbol": "SPCS3",
  "gene_name": "Signal peptidase complex subunit 3"
}